{
  "term_id": "GO:0045505",
  "term_label": "dynein intermediate chain binding",
  "gene_name": "Cytoplasmic dynein 2 heavy chain 1",
  "gene_symbol": "DYNC2H1",
  "gene": "UniProtKB:Q8NCM8"
}